{
  "term_id": "GO:0016323",
  "gene_name": "ATP-binding cassette sub-family C member 6",
  "gene": "UniProtKB:O95255",
  "gene_symbol": "ABCC6",
  "term_label": "basolateral plasma membrane"
}